galectin complex [GO:1990724] (cellular component) Note: An example of this is Galectin-1 in human (P09382) in PMID:15476813 (inferred from physical interaction). Relationships: is_a protein complex involved in cell-cell adhesion [GO:0098635] Definition: A homodimeric protein complex that is capable of binding a range of carbohydrates and is involved in anti-inflammatory and pro-apoptotic processes. References: PMID:15476813, PMID:18777589, PMID:8262940 Sources: GOC:bhm Also known as: galectin-1 complex, galectin-2 complex